{
  "gene": "UniProtKB:P13637",
  "gene_name": "Sodium_potassium-transporting ATPase subunit alpha-3",
  "term_id": "GO:0005886",
  "gene_symbol": "ATP1A3",
  "term_label": "plasma membrane"
}